{
  "gene": "UniProtKB:P22492",
  "gene_name": "Histone H1t",
  "term_id": "GO:0030261",
  "gene_symbol": "H1-6",
  "term_label": "chromosome condensation"
}